{
  "term_label": "protein-macromolecule adaptor activity",
  "term_id": "GO:0030674",
  "gene_symbol": "LIN7A",
  "gene_name": "Protein lin-7 homolog A",
  "gene": "UniProtKB:O14910"
}